{
  "gene_name": "BCL2_adenovirus E1B 19 kDa protein-interacting protein 3-like",
  "gene": "UniProtKB:O60238",
  "term_label": "nucleus",
  "term_id": "GO:0005634",
  "gene_symbol": "BNIP3L"
}